{
  "term_label": "Unknown molecular function",
  "gene_name": "Leucine-rich repeat and transmembrane domain-containing protein 2",
  "term_id": "UNKNOWN:0001",
  "gene_symbol": "LRTM2",
  "gene": "UniProtKB:Q8N967"
}